{
  "gene_symbol": "ZNF300",
  "term_label": "RNA polymerase II cis-regulatory region sequence-specific DNA binding",
  "gene_name": "Zinc finger protein 300",
  "term_id": "GO:0000978",
  "gene": "UniProtKB:Q96RE9"
}